{
  "gene": "UniProtKB:A0A1W2PPE2",
  "gene_symbol": "TAF11L4",
  "term_id": "GO:0005669",
  "gene_name": "TATA-box-binding protein-associated factor 11-like protein 4",
  "term_label": "transcription factor TFIID complex"
}